{
  "gene_name": "Receptor activity-modifying protein 2",
  "term_id": "GO:0001525",
  "gene_symbol": "RAMP2",
  "gene": "UniProtKB:O60895",
  "term_label": "angiogenesis"
}